{
  "gene_symbol": "CDCA3",
  "term_id": "UNKNOWN:0003",
  "gene_name": "Cell division cycle-associated protein 3",
  "gene": "UniProtKB:Q99618",
  "term_label": "Unknown cellular component"
}